{
  "gene": "UniProtKB:Q8WZ94",
  "gene_name": "Olfactory receptor 5P3",
  "gene_symbol": "OR5P3",
  "term_label": "odorant binding",
  "term_id": "GO:0005549"
}